{
  "gene_symbol": "H4C16",
  "gene_name": "Histone H4",
  "term_label": "structural constituent of chromatin",
  "term_id": "GO:0030527",
  "gene": "UniProtKB:P62805"
}